{
  "gene_symbol": "FAM227A",
  "term_label": "Unknown cellular component",
  "gene": "UniProtKB:F5H4B4",
  "term_id": "UNKNOWN:0003",
  "gene_name": "Protein FAM227A"
}